purine deoxyribonucleotide biosynthetic process [GO:0009153] (biological process) Definition: The chemical reactions and pathways resulting in the formation of purine deoxyribonucleotide, a compound consisting of deoxyribonucleoside (a purine base linked to a deoxyribose sugar) esterified with a phosphate group at either the 3' or 5'-hydroxyl group of the sugar. Relationships: is a type of GO:0006164; is a type of purine deoxyribonucleotide metabolic process [GO:0009151]; is a type of GO:0009265 Also known as: purine deoxyribonucleotide anabolism, purine deoxyribonucleotide biosynthesis, purine deoxyribonucleotide formation, purine deoxyribonucleotide synthesis Subtypes: dAMP biosynthetic process [GO:0006170], dADP biosynthetic process [GO:0006173], dATP biosynthetic process [GO:0006175], dGMP biosynthetic process [GO:0006181], dGDP biosynthetic process [GO:0006185], dGTP biosynthetic process [GO:0046071], purine deoxyribonucleotide salvage [GO:0106381] Sources: GOC:go_curators, ISBN:0198506732